{
  "gene": "UniProtKB:O43918",
  "gene_symbol": "AIRE",
  "term_label": "nucleus",
  "gene_name": "Autoimmune regulator",
  "term_id": "GO:0005634"
}